{
  "gene": "UniProtKB:A0A087WYE8",
  "gene_symbol": "IGHV1OR21-1",
  "term_label": "immunoglobulin mediated immune response",
  "gene_name": "Immunoglobulin heavy variable 1_OR21-1 (non-functional) (Fragment)",
  "term_id": "GO:0016064"
}